{
  "gene_symbol": "TNF",
  "gene": "UniProtKB:P01375",
  "gene_name": "Tumor necrosis factor",
  "term_label": "extracellular space",
  "term_id": "GO:0005615"
}